{
  "gene_symbol": "KIR3DX1",
  "gene": "UniProtKB:Q9H7L2",
  "term_label": "immune receptor activity",
  "gene_name": "Putative killer cell immunoglobulin-like receptor-like protein KIR3DX1",
  "term_id": "GO:0140375"
}